muscular septum morphogenesis [GO:0003150] (biological process) Relationships: is a type of muscle tissue morphogenesis [GO:0060415]; is part of ventricular septum morphogenesis [GO:0060412] Definition: The process in which the muscular septum is generated and organized. The muscular septum is the lower part of the ventricular septum. Sources: GOC:mtg_heart